left-handed Z-DNA binding [GO:0003692] (molecular function) Definition: Binding to DNA in the Z form, i.e. a left-handed helix in which the phosphate backbone zigzags. Relationships: is a type of GO:0003690 Sources: ISBN:0716720094